{
  "term_label": "condensed nuclear chromosome",
  "gene_symbol": "IHO1",
  "gene": "UniProtKB:Q8IYA8",
  "gene_name": "Interactor of HORMAD1 protein 1",
  "term_id": "GO:0000794"
}